{
  "gene_symbol": "SMARCAL1",
  "term_label": "DNA repair",
  "term_id": "GO:0006281",
  "gene": "UniProtKB:Q9NZC9",
  "gene_name": "SWI_SNF-related matrix-associated actin-dependent regulator of chromatin subfamily A-like protein 1"
}